regulation of trophoblast cell migration [GO:1901163] (biological process) Subtypes: GO:1901164, GO:1901165 Relationships: is a type of GO:0030334; regulates trophoblast cell migration [GO:0061450] Sources: GOC:BHF, GOC:TermGenie Definition: Any process that modulates the frequency, rate or extent of trophoblast cell migration.